{
  "gene": "UniProtKB:Q9UID3",
  "term_label": "retrograde transport, endosome to Golgi",
  "gene_symbol": "VPS51",
  "term_id": "GO:0042147",
  "gene_name": "Vacuolar protein sorting-associated protein 51 homolog"
}